gamma DNA polymerase complex [GO:0005760] (cellular component) Definition: A DNA polymerase complex consisting of a large subunit, responsible for the catalytic activities, and a small accessory subunit. Functions in the replication and repair of mitochondrial DNA. Relationships: is a type of DNA polymerase complex [GO:0042575]; is a type of GO:0098798; is part of GO:0005759 References: PMID:12045093 Sources: GOC:jl